{
  "term_id": "GO:0000030",
  "gene_name": "Putative C-mannosyltransferase DPY19L2P2",
  "gene_symbol": "DPY19L2P2",
  "term_label": "mannosyltransferase activity",
  "gene": "UniProtKB:Q6ZN68"
}